{
  "gene_symbol": "COQ3",
  "term_label": "3-demethylubiquinol 3-O-methyltransferase activity",
  "term_id": "GO:0061542",
  "gene": "UniProtKB:Q9NZJ6",
  "gene_name": "Ubiquinone biosynthesis O-methyltransferase, mitochondrial"
}